{
  "gene": "UniProtKB:O43752",
  "gene_symbol": "STX6",
  "gene_name": "Syntaxin-6",
  "term_id": "GO:0005484",
  "term_label": "SNAP receptor activity"
}